{
  "gene_symbol": "NUPR2",
  "gene": "UniProtKB:A6NF83",
  "gene_name": "Nuclear protein 2",
  "term_id": "UNKNOWN:0001",
  "term_label": "Unknown molecular function"
}